{
  "gene": "UniProtKB:Q13094",
  "term_id": "GO:0005737",
  "gene_name": "Lymphocyte cytosolic protein 2",
  "term_label": "cytoplasm",
  "gene_symbol": "LCP2"
}